{
  "term_label": "beta-catenin binding",
  "gene_name": "Cadherin-18",
  "gene": "UniProtKB:Q13634",
  "term_id": "GO:0008013",
  "gene_symbol": "CDH18"
}